{
  "term_id": "UNKNOWN:0002",
  "term_label": "Unknown biological process",
  "gene": "UniProtKB:A2A3L6",
  "gene_name": "Tetratricopeptide repeat protein 24",
  "gene_symbol": "TTC24"
}